{
  "gene_name": "Beta-defensin 132",
  "term_label": "extracellular space",
  "gene": "UniProtKB:Q7Z7B7",
  "gene_symbol": "DEFB132",
  "term_id": "GO:0005615"
}